mystery cell differentiation [GO:0008583] (biological process) Relationships: is a type of cell differentiation [GO:0030154]; is part of compound eye morphogenesis [GO:0001745] Definition: The process in which an undifferentiated cell acquires the features of a mystery cell. The mystery cells are a precluster of cells that emerge from the compound eye morphogenetic furrow, normally positioned between R3 and R4. They then disappear into the surrounding pool of undifferentiated cells and have no known fate in the mature ommatidium. An example of this process is found in Drosophila melanogaster. References: PMID:1295747 Sources: ISBN:0632030488